{
  "term_label": "Unknown cellular component",
  "gene": "UniProtKB:Q13564",
  "gene_symbol": "NAE1",
  "gene_name": "NEDD8-activating enzyme E1 regulatory subunit",
  "term_id": "UNKNOWN:0003"
}